{
  "gene": "UniProtKB:Q14994",
  "gene_name": "Nuclear receptor subfamily 1 group I member 3",
  "term_label": "RNA polymerase II cis-regulatory region sequence-specific DNA binding",
  "gene_symbol": "NR1I3",
  "term_id": "GO:0000978"
}